cell migration involved in heart formation [GO:0060974] (biological process) Definition: The orderly movement of a cell from one site to another that contribute to the formation of the heart. The initial heart structure is made up of mesoderm-derived heart progenitor cells and neural crest-derived cells. Sources: GOC:mtg_heart Relationships: is a type of GO:0060973; is part of heart formation [GO:0060914] Subtypes: neural crest cell migration involved in heart formation [GO:0003147], cardioblast migration [GO:0003260]